{
  "term_label": "cytoplasmic side of plasma membrane",
  "gene_name": "TNF receptor-associated factor 3",
  "term_id": "GO:0009898",
  "gene": "UniProtKB:Q13114",
  "gene_symbol": "TRAF3"
}